regulation of adult somatic muscle development [GO:0062226] (biological process) Definition: Any process that modulates the rate, frequency or extent of adult somatic muscle development. References: PMID:16643882, PMID:25758712 Subtypes: positive regulation of adult somatic muscle development [GO:0062227], negative regulation of adult somatic muscle development [GO:0062228] Relationships: is a type of GO:0062223; regulates adult somatic muscle development [GO:0007527]